{
  "term_id": "GO:0033691",
  "gene": "UniProtKB:P20138",
  "gene_symbol": "CD33",
  "term_label": "sialic acid binding",
  "gene_name": "Myeloid cell surface antigen CD33"
}